{
  "gene": "UniProtKB:Q96LT7",
  "gene_symbol": "C9orf72",
  "term_label": "autophagosome",
  "term_id": "GO:0005776",
  "gene_name": "Guanine nucleotide exchange factor C9orf72"
}